engulfment of apoptotic cell [GO:0043652] (biological process) References: PMID:15536015 Sources: GOC:rk Regulation: regulated by regulation of engulfment of apoptotic cell [GO:1901074]; negatively regulated by negative regulation of engulfment of apoptotic cell [GO:1901075]; positively regulated by positive regulation of engulfment of apoptotic cell [GO:1901076] Relationships: is a type of phagocytosis, engulfment [GO:0006911]; is part of apoptotic cell clearance [GO:0043277] Note: This term should be used to annotate gene products from the engulfing cell that facilitate phagocytosis of apoptotic cells. It should not be mistaken with GO:0070782 'phosphatidylserine exposure on apoptotic cell surface', a process occurring in apoptotic cells that acts as a signal for engulfing cells. If gene products involved in such instances of phosphatidylserine exposure are shown to have a positive effect on engulfment, they may be annotated to GO:1901076 'positive regulation of engulfment of apoptotic cell'. Definition: The removal of the apoptotic cell by phagocytosis, by a neighboring cell or by a phagocyte. Also known as: engulfment of apoptotic cell corpse, engulfment of cell corpse